{
  "term_label": "Unknown biological process",
  "gene_symbol": "MYBPHL",
  "term_id": "UNKNOWN:0002",
  "gene": "UniProtKB:A2RUH7",
  "gene_name": "Myosin-binding protein H-like"
}